chloroplast starch grain [GO:0009569] (cellular component) Also known as: chloroplast starch granule Relationships: is_a GO:0043036; is part of GO:0009507 Definition: Plant storage body for amylose and amylopectin, 1-100um in diameter, and located in chloroplasts. Also contains small amounts of enzymes, amino acids, lipids and nucleic acids. The shape of the grain varies widely amongst species, but is often spherical or disk-shaped. Sources: GOC:jl, ISBN:0198506732